{
  "term_label": "Unknown molecular function",
  "term_id": "UNKNOWN:0001",
  "gene": "UniProtKB:Q9H2P9",
  "gene_symbol": "DPH5",
  "gene_name": "Diphthine methyl ester synthase"
}